{
  "term_label": "Unknown molecular function",
  "gene_symbol": "SDHB",
  "term_id": "UNKNOWN:0001",
  "gene": "UniProtKB:P21912",
  "gene_name": "Succinate dehydrogenase [ubiquinone] iron-sulfur subunit, mitochondrial"
}